positive regulation of apolipoprotein A-I-mediated signaling pathway [GO:1905096] (biological process) References: PMID:25084135 Sources: GOC:BHF, GOC:BHF_miRNA, GOC:TermGenie, GOC:bc, GO_REF:0000058 Also known as: positive regulation of apolipoprotein A-I-mediated signalling pathway, up regulation of apolipoprotein A-I-mediated signaling pathway, up regulation of apolipoprotein A-I-mediated signalling pathway, up-regulation of apolipoprotein A-I-mediated signaling pathway, up-regulation of apolipoprotein A-I-mediated signalling pathway, upregulation of apolipoprotein A-I-mediated signaling pathway, upregulation of apolipoprotein A-I-mediated signalling pathway, activation of apolipoprotein A-I-mediated signaling pathway, activation of apolipoprotein A-I-mediated signalling pathway Definition: Any process that activates or increases the frequency, rate or extent of apolipoprotein A-I-mediated signaling pathway. Relationships: is a type of GO:0009967; is a type of regulation of apolipoprotein A-I-mediated signaling pathway [GO:1905094]; positively regulates apolipoprotein A-I-mediated signaling pathway [GO:0038027]